{
  "term_label": "external side of plasma membrane",
  "gene_symbol": "CD86",
  "gene_name": "T-lymphocyte activation antigen CD86",
  "term_id": "GO:0009897",
  "gene": "UniProtKB:P42081"
}